{
  "gene": "UniProtKB:P55347",
  "gene_name": "Homeobox protein PKNOX1",
  "gene_symbol": "PKNOX1",
  "term_label": "nucleus",
  "term_id": "GO:0005634"
}